{
  "gene": "UniProtKB:O14668",
  "term_label": "proteolysis",
  "term_id": "GO:0006508",
  "gene_name": "Transmembrane gamma-carboxyglutamic acid protein 1",
  "gene_symbol": "PRRG1"
}